toluene-containing compound catabolic process [GO:0072491] (biological process) Subtypes: p-cymene catabolic process [GO:0019334], GO:0042203, orcinol catabolic process [GO:0042209], cresol catabolic process [GO:0046199], nitrotoluene catabolic process [GO:0046263], toluene-4-sulfonate catabolic process [GO:0046269] Sources: GOC:mah Relationships: is a type of catabolic process [GO:0009056]; is a type of benzene-containing compound metabolic process [GO:0042537] Also known as: toluene and derivative catabolic process, toluene-containing compound breakdown, toluene-containing compound catabolism, toluene-containing compound degradation Definition: The chemical reactions and pathways resulting in the breakdown of toluene, methylbenzene (formula C7H8), or any of its derivatives.